sulfite export across plasma membrane [GO:0160244] (biological process) Relationships: is a type of sulfite transmembrane transport [GO:0000316]; is a type of export across plasma membrane [GO:0140115]; is part of detoxification of sulfite [GO:0160245] Also known as: sulfite efflux References: PMID:17322211, PMID:30859719 Definition: The directed movement of sulfite from inside of a cell, across the plasma membrane and into the extracellular region.